{
  "term_label": "plasma membrane",
  "gene": "UniProtKB:A0A539",
  "gene_symbol": "TRBV4-2",
  "gene_name": "T cell receptor beta variable 4-2",
  "term_id": "GO:0005886"
}